negative regulation of lipid binding [GO:1900131] (biological process) Relationships: is a type of negative regulation of binding [GO:0051100]; negatively regulates lipid binding [GO:0008289] Also known as: down regulation of lipid binding, down-regulation of lipid binding, downregulation of lipid binding, inhibition of lipid binding Definition: Any process that stops, prevents or reduces the frequency, rate or extent of lipid binding. Sources: GOC:TermGenie, GOC:pm